{
  "gene_name": "Interleukin-17 receptor B",
  "term_label": "Unknown biological process",
  "term_id": "UNKNOWN:0002",
  "gene": "UniProtKB:Q9NRM6",
  "gene_symbol": "IL17RB"
}